{
  "gene": "UniProtKB:O60462",
  "gene_name": "Neuropilin-2",
  "term_label": "postsynaptic membrane",
  "gene_symbol": "NRP2",
  "term_id": "GO:0045211"
}